{
  "gene_name": "Lipase member H",
  "term_label": "extracellular space",
  "gene_symbol": "LIPH",
  "gene": "UniProtKB:Q8WWY8",
  "term_id": "GO:0005615"
}